{
  "term_id": "GO:0005783",
  "gene_symbol": "ANKRD13C",
  "gene": "UniProtKB:Q8N6S4",
  "term_label": "endoplasmic reticulum",
  "gene_name": "Ankyrin repeat domain-containing protein 13C"
}